{
  "gene_symbol": "KCNC3",
  "gene": "UniProtKB:Q14003",
  "term_label": "postsynaptic membrane",
  "gene_name": "Potassium voltage-gated channel subfamily C member 3",
  "term_id": "GO:0045211"
}